{
  "gene_name": "Endogenous retrovirus group K member 25 Pol protein",
  "gene_symbol": "ERVK-25",
  "term_id": "GO:0035613",
  "term_label": "RNA stem-loop binding",
  "gene": "UniProtKB:P63136"
}